{
  "term_label": "Unknown molecular function",
  "gene_symbol": "LINC01590",
  "gene": "UniProtKB:Q5TEZ4",
  "gene_name": "Putative uncharacterized protein encoded by LINC01590",
  "term_id": "UNKNOWN:0001"
}